epithelial to mesenchymal transition [GO:0001837] (biological process) Relationships: is a type of mesenchymal cell differentiation [GO:0048762] References: PMID:14701881 Sources: GOC:dph Subtypes: GO:0003347, neural crest formation [GO:0014029], cardiac epithelial to mesenchymal transition [GO:0060317], mesodermal to mesenchymal transition involved in gastrulation [GO:0060809], clearance of cells from fusion plate by epithelial to mesenchymal transition [GO:0060886] Also known as: EMT, epithelial-mesenchymal transition, mesenchymal cell differentiation from epithelial cell Regulation: regulated by GO:0010717; positively regulated by positive regulation of epithelial to mesenchymal transition [GO:0010718]; negatively regulated by negative regulation of epithelial to mesenchymal transition [GO:0010719] Definition: A transition where an epithelial cell loses apical/basolateral polarity, severs intercellular adhesive junctions, degrades basement membrane components and becomes a migratory mesenchymal cell.